{
  "gene": "UniProtKB:P12273",
  "term_id": "GO:0005615",
  "gene_name": "Prolactin-inducible protein",
  "gene_symbol": "PIP",
  "term_label": "extracellular space"
}